{
  "term_label": "odorant binding",
  "gene": "UniProtKB:Q8NH90",
  "term_id": "GO:0005549",
  "gene_name": "Olfactory receptor 5AK2",
  "gene_symbol": "OR5AK2"
}